{
  "gene_name": "DNA dC-dU-editing enzyme APOBEC-3A",
  "term_id": "GO:0005737",
  "gene_symbol": "APOBEC3A",
  "term_label": "cytoplasm",
  "gene": "UniProtKB:P31941"
}